{
  "term_id": "GO:0031175",
  "term_label": "neuron projection development",
  "gene": "UniProtKB:O60542",
  "gene_name": "Persephin",
  "gene_symbol": "PSPN"
}